{
  "gene": "UniProtKB:Q99645",
  "term_id": "GO:0031012",
  "term_label": "extracellular matrix",
  "gene_name": "Epiphycan",
  "gene_symbol": "EPYC"
}